{
  "term_id": "UNKNOWN:0003",
  "gene_symbol": "NXPH4",
  "term_label": "Unknown cellular component",
  "gene": "UniProtKB:O95158",
  "gene_name": "Neurexophilin-4"
}